{
  "gene": "UniProtKB:Q9HCX4",
  "gene_symbol": "TRPC7",
  "term_label": "store-operated calcium channel activity",
  "term_id": "GO:0015279",
  "gene_name": "Short transient receptor potential channel 7"
}